{
  "gene_symbol": "HEMGN",
  "gene": "UniProtKB:Q9BXL5",
  "term_label": "regulation of osteoblast differentiation",
  "gene_name": "Hemogen",
  "term_id": "GO:0045667"
}